{
  "term_label": "Unknown cellular component",
  "gene_name": "Uncharacterized protein C17orf100",
  "gene": "UniProtKB:A8MU93",
  "gene_symbol": "C17orf100",
  "term_id": "UNKNOWN:0003"
}